growth factor signaling initiating cell movement involved in cerebral cortex radial glia guided migration [GO:0021811] (biological process) References: PMID:12626695 Sources: GOC:cls, GOC:dgh, GOC:dph, GOC:jid, GO_REF:0000021 Relationships: is a type of motogenic signaling initiating cell movement in cerebral cortex [GO:0021807] Also known as: growth factor signaling initiating cell movement involved in cerebral cortex glial-mediated radial migration, growth factor signalling initiating cell movement involved in cerebral cortex glial-mediated radial migration Definition: Signaling between growth factors and their receptors that results in the start of cell movement, where this process is involved in glial-mediated radial migration in the cerebral cortex.